regulation of translational initiation by eIF2 alpha phosphorylation [GO:0010998] (biological process) Subtypes: eiF2alpha phosphorylation in response to endoplasmic reticulum stress [GO:0036492] Definition: Any process that modulates the frequency, rate or extent of translation initiation in response to stress by the phosphorylation of eIF2 alpha. Note: Consider also annotating to 'eukaryotic translation initiation factor 2alpha kinase activity ; GO:0004694'. Also known as: eIF2 alpha phosphorylation in response to stress, regulation of translational initiation by eIF2 alpha phosphorylation in response to stress Regulation: regulated by regulation of eIF2 alpha phosphorylation by heme [GO:0010999]; regulated by regulation of eIF2 alpha phosphorylation by dsRNA [GO:0060735] Sources: GOC:BHF, GOC:dph, GOC:hjd, GOC:tb Relationships: is a type of protein phosphorylation [GO:0006468]; is a type of regulation of translational initiation in response to stress [GO:0043558]